{
  "term_id": "UNKNOWN:0002",
  "gene": "UniProtKB:Q147U7",
  "gene_name": "Single-pass membrane and coiled-coil domain-containing protein 1",
  "term_label": "Unknown biological process",
  "gene_symbol": "SMCO1"
}